{
  "gene_name": "Immunoglobulin heavy constant gamma 2",
  "term_label": "antibacterial humoral response",
  "term_id": "GO:0019731",
  "gene": "UniProtKB:P01859",
  "gene_symbol": "IGHG2"
}